negative regulation of single-species biofilm formation [GO:1900191] (biological process) Also known as: down regulation of single-species biofilm formation, down-regulation of single-species biofilm formation, downregulation of single-species biofilm formation, inhibition of single-species biofilm formation Relationships: is a type of negative regulation of cellular process [GO:0048523]; is a type of GO:1900190; negatively regulates GO:0044010 Definition: Any process that stops, prevents or reduces the frequency, rate or extent of single-species biofilm formation. Subtypes: negative regulation of single-species biofilm formation in or on host organism [GO:1900229], negative regulation of single-species biofilm formation on inanimate substrate [GO:1900232] Sources: GOC:TermGenie, GOC:di